{
  "gene": "UniProtKB:Q9UGP5",
  "term_label": "nucleus",
  "term_id": "GO:0005634",
  "gene_name": "DNA polymerase lambda",
  "gene_symbol": "POLL"
}